positive regulation of sulfite transmembrane transport [GO:1900072] (biological process) Relationships: is a type of positive regulation of transmembrane transport [GO:0034764]; is a type of GO:1900071; positively regulates sulfite transmembrane transport [GO:0000316] Also known as: positive regulation of sulfite transport, positive regulation of sulphite transport, up regulation of sulphite transport, up-regulation of sulphite transport, upregulation of sulphite transport, activation of sulfite transport, activation of sulphite transport, up regulation of sulfite transport, up-regulation of sulfite transport, upregulation of sulfite transport References: PMID:10234785, PMID:10870099 Sources: GOC:TermGenie Definition: Any process that activates or increases the frequency, rate or extent of sulfite transmembrane transport.